{
  "term_id": "GO:0007035",
  "term_label": "vacuolar acidification",
  "gene": "UniProtKB:Q9Y5K8",
  "gene_name": "V-type proton ATPase subunit D",
  "gene_symbol": "ATP6V1D"
}